{
  "term_id": "GO:0005865",
  "gene": "UniProtKB:P28289",
  "term_label": "striated muscle thin filament",
  "gene_symbol": "TMOD1",
  "gene_name": "Tropomodulin-1"
}